{
  "gene_symbol": "KRTAP4-6",
  "term_id": "UNKNOWN:0003",
  "gene_name": "Keratin-associated protein 4-6",
  "gene": "UniProtKB:Q9BYQ5",
  "term_label": "Unknown cellular component"
}